{
  "gene_symbol": "HMGB2",
  "gene_name": "High mobility group protein B2",
  "term_id": "GO:0005634",
  "gene": "UniProtKB:P26583",
  "term_label": "nucleus"
}